U12-type prespliceosome [GO:0071015] (cellular component) References: PMID:10197985, PMID:16201866 Sources: GOC:ab, GOC:krc, GOC:mah Also known as: minor prespliceosome, AT-AC prespliceosome, mammalian U12-type spliceosomal complex A, yeast U12-type spliceosomal complex B Definition: A spliceosomal complex that is formed by the cooperative binding of the heterodimeric U11/U12 snRNP to the 5' splice site and the branch point sequence. The U12-type prespliceosome includes many proteins in addition to those found in the U11/U12 heterodimeric snRNPs. Commitment to a given pair of 5' and 3' splice sites occurs at the time of prespliceosome formation. Relationships: is a type of U12-type spliceosomal complex [GO:0005689]; is a type of prespliceosome [GO:0071010]; has part U11/U12 snRNP [GO:0034693]